{
  "gene": "UniProtKB:O15318",
  "term_id": "GO:0005666",
  "gene_name": "DNA-directed RNA polymerase III subunit RPC7",
  "term_label": "RNA polymerase III complex",
  "gene_symbol": "POLR3G"
}